mating-type region heterochromatin [GO:0031934] (cellular component) Sources: GOC:mah Relationships: is a type of GO:0000792 Definition: Heterochromatic regions of the chromosome found at silenced mating-type loci.